{
  "gene_name": "Zinc transporter ZIP6",
  "term_label": "monoatomic cation:bicarbonate symporter activity",
  "gene_symbol": "SLC39A6",
  "term_id": "GO:0140410",
  "gene": "UniProtKB:Q13433"
}